{
  "gene_name": "RNA-binding protein MEX3D",
  "gene_symbol": "MEX3D",
  "gene": "UniProtKB:Q86XN8",
  "term_label": "Unknown cellular component",
  "term_id": "UNKNOWN:0003"
}